{
  "gene_name": "Ras-related protein Rab-12",
  "gene": "UniProtKB:Q6IQ22",
  "gene_symbol": "RAB12",
  "term_label": "trans-Golgi network transport vesicle",
  "term_id": "GO:0030140"
}